piRNA processing [GO:0034587] (biological process) Relationships: is a type of regulatory ncRNA processing [GO:0070918] Also known as: PIWI-associated RNA biogenesis, PIWI-associated RNA processing, piRNA biogenesis, Piwi-associated RNA biosynthetic process, Piwi-associated RNA metabolic process, piRNA biosynthetic process, piRNA metabolic process, piRNA metabolism References: PMID:23329111, PMID:24696457, PMID:34724117 Sources: GOC:kmv Definition: A process leading to the generation of a functional piRNA. piRNAs (Piwi-associated RNAs) are a class of 24- to 30-nucleotide RNAs derived from repeat or complex DNA sequence elements and processed by a Dicer-independent mechanism. Subtypes: secondary piRNA processing [GO:0140965], GO:0140990